{
  "gene_symbol": "TMEM207",
  "term_id": "UNKNOWN:0003",
  "gene": "UniProtKB:Q6UWW9",
  "term_label": "Unknown cellular component",
  "gene_name": "Transmembrane protein 207"
}